chromaffin granule lumen [GO:0034466] (cellular component) Relationships: is a type of secretory granule lumen [GO:0034774]; is part of chromaffin granule [GO:0042583] Definition: The volume enclosed by the membrane of a chromaffin granule. Sources: GOC:rph